{
  "gene_name": "Golgin subfamily A member 7",
  "term_id": "GO:0043001",
  "term_label": "Golgi to plasma membrane protein transport",
  "gene_symbol": "GOLGA7",
  "gene": "UniProtKB:Q7Z5G4"
}